bub1-bub3 complex [GO:1990298] (cellular component) References: PMID:22521786 Relationships: is a type of protein-containing complex [GO:0032991] Definition: Protein complex that associates with the kinetochores.